regulation of mitochondrial DNA replication [GO:0090296] (biological process) Relationships: is a type of regulation of DNA-templated DNA replication [GO:0090329]; is a type of regulation of mitochondrial DNA metabolic process [GO:1901858]; regulates GO:0006264 Sources: GOC:tb Subtypes: GO:0090297, negative regulation of mitochondrial DNA replication [GO:0090298] Definition: Any process that modulates the rate, frequency or extent of the process in which new strands of DNA are synthesized in the mitochondrion. Also known as: regulation of mitochondrial DNA synthesis